{
  "gene": "UniProtKB:Q3SXM0",
  "gene_symbol": "DCAF4L1",
  "term_label": "Cul4-RING E3 ubiquitin ligase complex",
  "gene_name": "DDB1- and CUL4-associated factor 4-like protein 1",
  "term_id": "GO:0080008"
}